keratinocyte activation [GO:0032980] (biological process) Relationships: is_a cell activation [GO:0001775] References: PMID:15737202 Sources: GOC:mah Definition: A change in the morphology or behavior of a keratinocyte resulting from exposure to an activating factor such as a cellular or soluble ligand. Upon activation, keratinocytes become migratory and hyperproliferative, and produce growth factors and cytokines.